{
  "term_label": "epigenetic regulation of gene expression",
  "gene": "UniProtKB:O60341",
  "gene_name": "Lysine-specific histone demethylase 1A",
  "gene_symbol": "KDM1A",
  "term_id": "GO:0040029"
}